{
  "term_label": "plasma membrane",
  "term_id": "GO:0005886",
  "gene": "UniProtKB:Q9UM47",
  "gene_name": "Neurogenic locus notch homolog protein 3",
  "gene_symbol": "NOTCH3"
}